{
  "term_label": "Unknown cellular component",
  "gene": "UniProtKB:Q6UY14",
  "gene_name": "ADAMTS-like protein 4",
  "gene_symbol": "ADAMTSL4",
  "term_id": "UNKNOWN:0003"
}